{
  "term_id": "GO:0005085",
  "gene_symbol": "CCZ1B",
  "term_label": "guanyl-nucleotide exchange factor activity",
  "gene_name": "Vacuolar fusion protein CCZ1 homolog B",
  "gene": "UniProtKB:P86790"
}